{
  "term_id": "UNKNOWN:0002",
  "gene_symbol": "CLCN4",
  "term_label": "Unknown biological process",
  "gene": "UniProtKB:P51793",
  "gene_name": "H(+)_Cl(-) exchange transporter 4"
}